response to antimycin A [GO:1901325] (BP) Subtypes: cellular response to antimycin A [GO:0072745] Definition: Any process that results in a change in state or activity of a cell or an organism (in terms of movement, secretion, enzyme production, gene expression, etc.) as a result of an antimycin A stimulus. Sources: GOC:TermGenie Relationships: is a type of response to nitrogen compound [GO:1901698]; is_a GO:1901700